{
  "term_label": "bile acid and bile salt transport",
  "gene_symbol": "SLC10A5",
  "gene_name": "Sodium_bile acid cotransporter 5",
  "gene": "UniProtKB:Q5PT55",
  "term_id": "GO:0015721"
}